{
  "term_id": "GO:0004993",
  "term_label": "G protein-coupled serotonin receptor activity",
  "gene_name": "5-hydroxytryptamine receptor 1D",
  "gene_symbol": "HTR1D",
  "gene": "UniProtKB:P28221"
}